{
  "term_label": "spindle assembly",
  "term_id": "GO:0051225",
  "gene_name": "Serine_threonine-protein phosphatase 2A 65 kDa regulatory subunit A alpha isoform",
  "gene": "UniProtKB:P30153",
  "gene_symbol": "PPP2R1A"
}